{
  "gene_name": "Leucine-rich repeat protein SHOC-2",
  "term_label": "cytoplasm",
  "term_id": "GO:0005737",
  "gene_symbol": "SHOC2",
  "gene": "UniProtKB:Q9UQ13"
}